positive regulation of cytoplasmic translation [GO:2000767] (biological process) Definition: Any process that activates or increases the frequency, rate or extent of cytoplasmic translation. Relationships: is_a positive regulation of translation [GO:0045727]; is a type of GO:2000765; positively regulates cytoplasmic translation [GO:0002181] Sources: GOC:obol